positive regulation of vernalization response [GO:0010220] (biological process) Sources: GOC:sm Also known as: up regulation of vernalization response, up-regulation of vernalization response, upregulation of vernalization response, activation of vernalization response, stimulation of vernalization response Definition: Any process that activates or induces the rate of the vernalization response, by which induction of flowering is normally caused by extended exposure to cold temperatures. Relationships: is a type of regulation of vernalization response [GO:0010219]; is a type of positive regulation of response to stimulus [GO:0048584]; positively regulates vernalization response [GO:0010048]